{
  "term_id": "GO:0070449",
  "term_label": "elongin complex",
  "gene": "UniProtKB:Q15370",
  "gene_symbol": "ELOB",
  "gene_name": "Elongin-B"
}